{
  "gene_name": "Procollagen galactosyltransferase 1",
  "gene": "UniProtKB:Q8NBJ5",
  "term_id": "UNKNOWN:0002",
  "gene_symbol": "COLGALT1",
  "term_label": "Unknown biological process"
}